alpha-ketoglutarate transmembrane transporter activity [GO:0015139] (MF) Subtypes: oxoglutarate:malate antiporter activity [GO:0015367], alpha-ketoglutarate:proton symporter activity [GO:0015532], citrate:2-oxoglutarate antiporter activity [GO:0180056] Also known as: 2-oxoglutarate transporter activity Definition: Enables the transfer of alpha-ketoglutarate from one side of a membrane to the other. Alpha-ketoglutarate (or oxoglutarate) is a compound with important roles in carbohydrate and amino acid metabolism, especially in transamination reactions and as a component of the TCA cycle. Sources: GOC:ai, ISBN:0198547684 Relationships: is a type of GO:0005310; is part of alpha-ketoglutarate transport [GO:0015742]